{
  "term_id": "GO:0005737",
  "gene_name": "Adenosine deaminase domain-containing protein 2",
  "term_label": "cytoplasm",
  "gene_symbol": "ADAD2",
  "gene": "UniProtKB:Q8NCV1"
}